{
  "term_id": "GO:0005525",
  "term_label": "GTP binding",
  "gene_name": "Ras-related protein Rab-30",
  "gene": "UniProtKB:Q15771",
  "gene_symbol": "RAB30"
}